{
  "gene": "UniProtKB:O60669",
  "term_id": "GO:0035879",
  "term_label": "plasma membrane lactate transport",
  "gene_symbol": "SLC16A7",
  "gene_name": "Monocarboxylate transporter 2"
}